{
  "term_id": "UNKNOWN:0001",
  "gene_name": "HIRA-interacting protein 3",
  "gene_symbol": "HIRIP3",
  "term_label": "Unknown molecular function",
  "gene": "UniProtKB:Q9BW71"
}